regulation of cellular response to gamma radiation [GO:1905843] (biological process) Subtypes: negative regulation of cellular response to gamma radiation [GO:1905844], positive regulation of cellular response to gamma radiation [GO:1905845] Relationships: is a type of regulation of cellular process [GO:0050794]; is a type of GO:2001228; regulates cellular response to gamma radiation [GO:0071480] Also known as: regulation of cellular response to gamma ray, regulation of cellular response to gamma-ray photon References: PMID:23505386 Sources: GOC:TermGenie, GO_REF:0000058 Definition: Any process that modulates the frequency, rate or extent of cellular response to gamma radiation.